{
  "term_id": "GO:0003713",
  "gene_name": "SERTA domain-containing protein 1",
  "term_label": "transcription coactivator activity",
  "gene_symbol": "SERTAD1",
  "gene": "UniProtKB:Q9UHV2"
}